triacyl lipopeptide binding [GO:0042497] (molecular function) Also known as: triacylated lipopeptide binding, bacterial triacyl lipopeptide binding, bacterial triacyl lipoprotein binding References: PMID:12077222, PMID:12524386, PMID:2757794 Sources: GOC:add Note: Note that bacterial lipopeptides are derived from bacterial lipoproteins, but the two terms are sometimes used interchangeably in the literature. Relationships: is a type of lipopeptide binding [GO:0071723] Definition: Binding to a lipopeptide containing a nonprotein moiety consisting of three acyl groups.